{
  "gene_name": "GEL complex subunit OPTI",
  "term_label": "Unknown biological process",
  "term_id": "UNKNOWN:0002",
  "gene_symbol": "RAB5IF",
  "gene": "UniProtKB:Q9BUV8"
}